{
  "term_id": "GO:0005737",
  "gene": "UniProtKB:Q15366",
  "gene_name": "Poly(rC)-binding protein 2",
  "term_label": "cytoplasm",
  "gene_symbol": "PCBP2"
}